leptotene [GO:0000237] (biological process) Definition: The cell cycle phase which is the first stage of prophase I in meiosis, and during which the chromosomes first become visible. Sources: GOC:mtg_cell_cycle Note: Note that this term should not be used for direct annotation. If you are trying to make an annotation to x phase, it is likely that the correct annotation is 'regulation of x/y phase transition' or to a process which occurs during the reported phase (i.e mitotic DNA replication for mitotic S-phase). To capture the phase when a specific location or process is observed, the phase term can be used in an annotation extension (PMID:24885854) applied to a cellular component term (with the relation exists_during) or a biological process term (with the relation happens_during). Relationships: is a type of meiosis I cell cycle phase [GO:0098764]; is part of meiotic prophase I [GO:0007128]